{
  "gene": "UniProtKB:Q99570",
  "gene_symbol": "PIK3R4",
  "term_label": "late endosome to vacuole transport",
  "gene_name": "Phosphoinositide 3-kinase regulatory subunit 4",
  "term_id": "GO:0045324"
}